{
  "term_label": "JUN kinase kinase kinase activity",
  "term_id": "GO:0004706",
  "gene_name": "Leucine-rich repeat serine_threonine-protein kinase 2",
  "gene_symbol": "LRRK2",
  "gene": "UniProtKB:Q5S007"
}